embryonic retina morphogenesis in camera-type eye [GO:0060059] (biological process) Sources: GOC:dgh, GOC:dph Relationships: is a type of embryonic morphogenesis [GO:0048598]; is part of GO:0060042 Definition: The process in which the anatomical structure of the retina is generated and organized in a camera-type eye during the embryonic life stage.